{
  "term_id": "GO:0031415",
  "term_label": "NatA complex",
  "gene": "UniProtKB:Q9BSU3",
  "gene_name": "N-alpha-acetyltransferase 11",
  "gene_symbol": "NAA11"
}